{
  "term_id": "UNKNOWN:0001",
  "gene_name": "Membrane-spanning 4-domains subfamily A member 6A",
  "gene": "UniProtKB:Q9H2W1",
  "term_label": "Unknown molecular function",
  "gene_symbol": "MS4A6A"
}